{
  "term_label": "SOSS complex",
  "term_id": "GO:0070876",
  "gene_name": "SOSS complex subunit B1",
  "gene_symbol": "NABP2",
  "gene": "UniProtKB:Q9BQ15"
}